{
  "gene": "UniProtKB:P14316",
  "gene_symbol": "IRF2",
  "term_id": "GO:0000981",
  "gene_name": "Interferon regulatory factor 2",
  "term_label": "DNA-binding transcription factor activity, RNA polymerase II-specific"
}